leptin receptor activity [GO:0038021] (MF) Relationships: is a type of GO:0004896; BFO_0000050 leptin-mediated signaling pathway [GO:0033210] References: PMID:9102398 Sources: GOC:bf, GOC:signaling, Wikipedia:Leptin_receptor Definition: Combining with the fat-cell specific hormone leptin and transmitting the signal from one side of the membrane to the other to initiate a change in cell activity.